{
  "gene_symbol": "TM4SF4",
  "gene_name": "Transmembrane 4 L6 family member 4",
  "term_label": "Unknown molecular function",
  "gene": "UniProtKB:P48230",
  "term_id": "UNKNOWN:0001"
}